peroxisome matrix targeting signal-2 binding [GO:0005053] (molecular function) References: PMID:11687502 Sources: GOC:mah Definition: Binding to a type 2 peroxisome targeting signal, a nonapeptide with a broad consensus sequence of (R/K)-(L/V/I)-(XXXXX)-(H/Q)-(L/A/F). Also known as: PTS2 binding, PTS2 receptor, peroxisomal targeting signal 2 (PTS2) binding, peroxisome targeting signal-2 binding, PEX7, peroxisome targeting signal-2 receptor Relationships: is a type of GO:0000268